{
  "term_id": "GO:0008528",
  "gene": "UniProtKB:Q02643",
  "term_label": "G protein-coupled peptide receptor activity",
  "gene_symbol": "GHRHR",
  "gene_name": "Growth hormone-releasing hormone receptor"
}